{
  "gene_symbol": "FGF5",
  "term_label": "regulation of cell migration",
  "gene": "UniProtKB:P12034",
  "term_id": "GO:0030334",
  "gene_name": "Fibroblast growth factor 5"
}